{
  "gene": "UniProtKB:Q6A162",
  "gene_name": "Keratin, type I cytoskeletal 40",
  "term_id": "GO:0045095",
  "gene_symbol": "KRT40",
  "term_label": "keratin filament"
}